negative regulation of type III hypersensitivity [GO:0001804] (biological process) Sources: GOC:add, ISBN:0781735149 Also known as: down regulation of type III hypersensitivity, down-regulation of type III hypersensitivity, downregulation of type III hypersensitivity, inhibition of type III hypersensitivity Relationships: is a type of regulation of type III hypersensitivity [GO:0001803]; is a type of negative regulation of hypersensitivity [GO:0002884]; is a type of negative regulation of myeloid leukocyte mediated immunity [GO:0002887]; is a type of negative regulation of immunoglobulin mediated immune response [GO:0002890]; negatively regulates type III hypersensitivity [GO:0001802] Definition: Any process that stops, prevents, or reduces the rate of type III hypersensitivity, a type of inflammatory response.